L-cysteine catabolic process via cystine, using cystine reductase [GO:0019455] (biological process) Definition: The chemical reactions and pathways resulting in the breakdown, via the compound cystine, of L-cysteine, catalyzed by the enzyme cystine reductase. Relationships: is a type of L-cysteine catabolic process via cystine [GO:0019453]; has part GO:0050456 Sources: GOC:jl Also known as: L-cysteine breakdown via cystine, using cystine reductase, L-cysteine degradation via cystine, using cystine reductase